{
  "gene_name": "1-acyl-sn-glycerol-3-phosphate acyltransferase beta",
  "term_id": "GO:0003841",
  "term_label": "1-acylglycerol-3-phosphate O-acyltransferase activity",
  "gene_symbol": "AGPAT2",
  "gene": "UniProtKB:O15120"
}